{
  "term_label": "collagen catabolic process",
  "gene_name": "Matrix metalloproteinase-26",
  "gene": "UniProtKB:Q9NRE1",
  "gene_symbol": "MMP26",
  "term_id": "GO:0030574"
}